mitochondrial DNA repair [GO:0043504] (biological process) References: PMID:12565799, PMID:15189144, PMID:16050976 Definition: The process of restoring mitochondrial DNA after damage. Relationships: is a type of GO:0006281; is a type of mitochondrial DNA metabolic process [GO:0032042]